skeletal muscle contraction [GO:0003009] (biological process) Relationships: is a type of striated muscle contraction [GO:0006941]; is part of GO:0050881 Definition: A process in which force is generated within skeletal muscle tissue, resulting in a change in muscle geometry. Force generation involves a chemo-mechanical energy conversion step that is carried out by the actin/myosin complex activity, which generates force through ATP hydrolysis. In the skeletal muscle, the muscle contraction takes advantage of an ordered sarcomeric structure and in most cases it is under voluntary control. Regulation: regulated by regulation of skeletal muscle contraction [GO:0014819] Sources: GOC:mtg_cardio, GOC:mtg_muscle Subtypes: GO:0003010, involuntary skeletal muscle contraction [GO:0003011]